{
  "gene_name": "Putative uncharacterized protein FLJ32756",
  "gene_symbol": "Q96M85",
  "term_label": "Unknown cellular component",
  "gene": "UniProtKB:Q96M85",
  "term_id": "UNKNOWN:0003"
}